{
  "gene_name": "Leucine zipper protein 2",
  "term_id": "UNKNOWN:0002",
  "term_label": "Unknown biological process",
  "gene": "UniProtKB:Q86TE4",
  "gene_symbol": "LUZP2"
}